{
  "gene_symbol": "DNAJC16",
  "term_label": "Unknown molecular function",
  "term_id": "UNKNOWN:0001",
  "gene_name": "DnaJ homolog subfamily C member 16",
  "gene": "UniProtKB:Q9Y2G8"
}